presynaptic endocytic zone membrane [GO:0098835] (cellular component) Relationships: is a type of synaptic membrane [GO:0097060]; is part of presynaptic membrane [GO:0042734]; is part of presynaptic endocytic zone [GO:0098833] Definition: The region of the presynaptic membrane that is part of the presynaptic endocytic zone - where synaptic vesicles are endocytosed and recycled following release. Sources: GOC:dos